{
  "gene_symbol": "BICDL1",
  "term_id": "GO:0055107",
  "gene": "UniProtKB:Q6ZP65",
  "term_label": "Golgi to secretory granule transport",
  "gene_name": "BICD family-like cargo adapter 1"
}